{
  "term_id": "GO:0045087",
  "gene_name": "Cathelicidin antimicrobial peptide",
  "gene": "UniProtKB:P49913",
  "gene_symbol": "CAMP",
  "term_label": "innate immune response"
}